{
  "gene_name": "Inositol polyphosphate 5-phosphatase OCRL",
  "term_label": "phosphatidylinositol-4,5-bisphosphate 5-phosphatase activity",
  "gene_symbol": "OCRL",
  "term_id": "GO:0004439",
  "gene": "UniProtKB:Q01968"
}